behavioral response to wounding [GO:0002210] (biological process) Definition: A behavioral response resulting from wounding. Also known as: behavioural response to wounding Relationships: is a type of behavior [GO:0007610]; is a type of response to wounding [GO:0009611] Sources: GOC:add, GO_REF:0000022